{
  "term_id": "GO:0005886",
  "gene_symbol": "STYK1",
  "gene": "UniProtKB:Q6J9G0",
  "term_label": "plasma membrane",
  "gene_name": "Tyrosine-protein kinase STYK1"
}